{
  "gene_name": "Cilia- and flagella-associated protein 20",
  "term_id": "GO:0036064",
  "gene": "UniProtKB:Q9Y6A4",
  "term_label": "ciliary basal body",
  "gene_symbol": "CFAP20"
}